G-protein gated monoatomic ion channel activity [GO:0099099] (MF) Definition: An ion channel activity that is gated by binding of a G-protein beta-gamma dimer. Also known as: G-protein gated ion channel activity Subtypes: G-protein gated monoatomic cation channel activity [GO:0099100] References: PMID:35704701 Sources: GOC:dos, Wikipedia:G_protein-gated_ion_channel Relationships: is a type of gated channel activity [GO:0022836]